{
  "term_label": "sex differentiation",
  "term_id": "GO:0007548",
  "gene_symbol": "DMRTA2",
  "gene": "UniProtKB:Q96SC8",
  "gene_name": "Doublesex- and mab-3-related transcription factor A2"
}